positive regulation of aortic smooth muscle cell differentiation [GO:1904831] (biological process) Relationships: is a type of regulation of aortic smooth muscle cell differentiation [GO:1904829]; is a type of positive regulation of vascular associated smooth muscle cell differentiation [GO:1905065]; positively regulates aortic smooth muscle cell differentiation [GO:0035887] Also known as: up regulation of aortic smooth muscle cell differentiation, up-regulation of aortic smooth muscle cell differentiation, upregulation of aortic smooth muscle cell differentiation, activation of aortic smooth muscle cell differentiation References: PMID:22034194 Sources: GOC:BHF, GOC:BHF_miRNA, GOC:TermGenie, GOC:rph, GO_REF:0000058 Definition: Any process that activates or increases the frequency, rate or extent of aortic smooth muscle cell differentiation.